ocelloid [GO:0097693] (cellular component) Definition: Eye-like subcellular structure found in dinoflagellates (a large group of single-celled eukaryotes). Consists of subcellular analogues to a cornea, lens, iris, and retina. Ocelloids are built from pre-existing organelles, including a cornea-like layer made of mitochondria and a retinal body made of anastomosing plastids. Relationships: is a type of GO:0043231; has part mitochondrion [GO:0005739]; has part GO:0009536 References: PMID:26131935 Sources: GOC:ar